{
  "term_id": "GO:0012505",
  "term_label": "endomembrane system",
  "gene_symbol": "RAB5A",
  "gene": "UniProtKB:P20339",
  "gene_name": "Ras-related protein Rab-5A"
}